{
  "term_label": "nuclear receptor activity",
  "gene_symbol": "NR2F6",
  "term_id": "GO:0004879",
  "gene": "UniProtKB:P10588",
  "gene_name": "Nuclear receptor subfamily 2 group F member 6"
}